{
  "term_id": "GO:0019941",
  "gene_symbol": "FAU",
  "gene_name": "Ubiquitin-like FUBI-ribosomal protein eS30 fusion protein",
  "gene": "UniProtKB:P62861",
  "term_label": "modification-dependent protein catabolic process"
}